{
  "gene": "UniProtKB:Q96SB3",
  "gene_symbol": "PPP1R9B",
  "term_id": "GO:0030425",
  "gene_name": "Neurabin-2",
  "term_label": "dendrite"
}